{
  "term_label": "Unknown cellular component",
  "term_id": "UNKNOWN:0003",
  "gene_symbol": "KIAA1210",
  "gene_name": "Acrosomal protein KIAA1210",
  "gene": "UniProtKB:Q9ULL0"
}